selenomethionine-tRNA ligase activity [GO:0098618] (molecular function) Definition: Catalysis of the reaction: ATP + L-selenomethionine + tRNA(Met) = AMP + diphosphate + selenomethionyl-tRNA(Met). References: PMID:16661668, PMID:16661782 Relationships: is a type of aminoacyl-tRNA ligase activity [GO:0004812]